perinuclear endoplasmic reticulum membrane [GO:1990578] (cellular component) Relationships: is a type of organelle membrane [GO:0031090]; is part of GO:0005789; is part of perinuclear endoplasmic reticulum [GO:0097038] References: PMID:25454947 Also known as: perinuclear ER membrane Definition: The membrane of the perinuclear endoplasmic reticulum, which is the portion of endoplasmic reticulum, the intracellular network of tubules and cisternae, that occurs near the nucleus.